{
  "gene_name": "Prostaglandin reductase 3",
  "term_label": "Unknown cellular component",
  "term_id": "UNKNOWN:0003",
  "gene_symbol": "PTGR3",
  "gene": "UniProtKB:Q8N4Q0"
}